{
  "term_label": "Unknown cellular component",
  "gene_name": "Terminal nucleotidyltransferase 5B",
  "gene": "UniProtKB:Q96A09",
  "gene_symbol": "TENT5B",
  "term_id": "UNKNOWN:0003"
}